regulation of carbohydrate utilization [GO:0043610] (biological process) Relationships: is a type of regulation of response to nutrient levels [GO:0032107]; regulates carbohydrate utilization [GO:0009758] Sources: GOC:jl Also known as: regulation of sugar utilization Definition: Any process that modulates the frequency, rate or extent of carbohydrate utilization.